{
  "gene_name": "Cell division cycle protein 123 homolog",
  "term_label": "Unknown molecular function",
  "gene_symbol": "CDC123",
  "gene": "UniProtKB:O75794",
  "term_id": "UNKNOWN:0001"
}